{
  "gene_name": "Heat shock 70 kDa protein 6",
  "gene_symbol": "HSPA6",
  "term_label": "cytosol",
  "gene": "UniProtKB:P17066",
  "term_id": "GO:0005829"
}